sulfur compound metabolic process [GO:0006790] (biological process) Subtypes: sulfur amino acid metabolic process [GO:0000096], sulfate assimilation [GO:0000103], GO:0006637, glutathione metabolic process [GO:0006749], GO:0006768, lipoate metabolic process [GO:0009106], mycothiol metabolic process [GO:0010126], coenzyme A metabolic process [GO:0015936], 4-carboxy-4'-sulfoazobenzene metabolic process [GO:0018887], cyclohexylsulfamate metabolic process [GO:0018892], GO:0018907, GO:0018909, GO:0018969, naphthalenesulfonate metabolic process [GO:0018984], polythionate oxidation [GO:0019416], sulfur oxidation [GO:0019417], GO:0019418, disproportionation of elemental sulfur [GO:0019422], GO:0019694, GO:0019760, S-methylmethionine metabolic process [GO:0033477], GO:0042316, GO:0042723, GO:0044272, sulfur compound catabolic process [GO:0044273], trypanothione metabolic process [GO:0046206], S-adenosylhomocysteine metabolic process [GO:0046498], GO:0046499, S-adenosylmethionine metabolic process [GO:0046500], GO:0046505, GO:0050427, dihydrolipoamide metabolic process [GO:0051068], sulfation [GO:0051923], thiazole metabolic process [GO:0052838], hydrogen sulfide metabolic process [GO:0070813], cephalosporin C metabolic process [GO:1901266], GO:2001131, methane biosynthetic process from 3-(methylthio)propionic acid [GO:2001132], methane biosynthetic process from methanethiol [GO:2001133] Relationships: is a type of metabolic process [GO:0008152] Definition: The chemical reactions and pathways involving the nonmetallic element sulfur or compounds that contain sulfur, such as the amino acids methionine and cysteine or the tripeptide glutathione. Regulation: regulated by regulation of sulfur metabolic process [GO:0042762] Also known as: sulfur metabolism, sulphur metabolic process, sulphur metabolism Sources: GOC:ai